canonical glycolysis [GO:0061621] (biological process) Definition: The glycolytic process that begins with the conversion of glucose to glucose-6-phosphate by glucokinase activity. Glycolytic processes are the chemical reactions and pathways resulting in the breakdown of a carbohydrate into pyruvate, with the concomitant production of a small amount of ATP. Sources: GOC:dph, ISBN:0201090910, ISBN:0879010479 Relationships: is a type of glycolytic process through glucose-6-phosphate [GO:0061620]; is a type of glucose catabolic process to pyruvate [GO:0061718]; has part GO:0004340; has part glyceraldehyde-3-phosphate dehydrogenase (NAD+) (phosphorylating) activity [GO:0004365]